{
  "gene": "UniProtKB:Q3LI64",
  "gene_name": "Keratin-associated protein 6-1",
  "term_label": "Unknown cellular component",
  "gene_symbol": "KRTAP6-1",
  "term_id": "UNKNOWN:0003"
}